{
  "gene_symbol": "PLSCR4",
  "gene": "UniProtKB:Q9NRQ2",
  "gene_name": "Phospholipid scramblase 4",
  "term_label": "plasma membrane phospholipid scrambling",
  "term_id": "GO:0017121"
}